{
  "gene_symbol": "ACOX1",
  "term_label": "flavin adenine dinucleotide binding",
  "gene_name": "Peroxisomal acyl-coenzyme A oxidase 1",
  "term_id": "GO:0050660",
  "gene": "UniProtKB:Q15067"
}